butyryl-CoA catabolic process [GO:0044580] (biological process) Also known as: butyryl-CoA catabolism Sources: GOC:jl Subtypes: butyryl-CoA catabolic process to butyrate [GO:0044581], butyryl-CoA catabolic process to butanol [GO:0044582] Definition: The chemical reactions a resulting in the resulting in the breakdown of butyryl-CoA. Relationships: is_a GO:0009062; is a type of fatty-acyl-CoA catabolic process [GO:0036115]